vestibular receptor cell stereocilium organization [GO:0060121] (biological process) Relationships: is a type of inner ear receptor cell stereocilium organization [GO:0060122]; is a type of neuron projection organization [GO:0106027]; is part of vestibular receptor cell morphogenesis [GO:0060116] Sources: GOC:dph Definition: A process that is carried out at the cellular level which results in the assembly, arrangement of constituent parts, or disassembly of a stereocilium. A stereocilium is an actin-based protrusion from the apical surface of vestibular hair cells. Also known as: vestibular hair cell stereocilium organization, vestibular receptor cell stereocilium organisation, vestibular receptor cell stereocilium organization and biogenesis